germ cell attraction [GO:0035232] (biological process) Definition: The directed movement of a germ cell from their site of production to the gonad, through the attraction of cells towards their target. References: PMID:12885551 Relationships: is a type of positive chemotaxis [GO:0050918]; is a type of cell chemotaxis [GO:0060326]; is part of germ cell migration [GO:0008354]